{
  "gene": "UniProtKB:O15060",
  "gene_symbol": "ZBTB39",
  "term_id": "GO:0001227",
  "gene_name": "Zinc finger and BTB domain-containing protein 39",
  "term_label": "DNA-binding transcription repressor activity, RNA polymerase II-specific"
}